{
  "term_id": "GO:0005102",
  "term_label": "signaling receptor binding",
  "gene": "UniProtKB:P09769",
  "gene_symbol": "FGR",
  "gene_name": "Tyrosine-protein kinase Fgr"
}